{
  "gene_name": "Olfactory receptor 4E1",
  "gene_symbol": "OR4E1",
  "term_label": "membrane",
  "term_id": "GO:0016020",
  "gene": "UniProtKB:P0C645"
}